{
  "gene_name": "Transmembrane gamma-carboxyglutamic acid protein 1",
  "gene_symbol": "PRRG1",
  "term_label": "extracellular space",
  "term_id": "GO:0005615",
  "gene": "UniProtKB:O14668"
}